{
  "gene_name": "POTE ankyrin domain family member I",
  "gene": "UniProtKB:P0CG38",
  "term_label": "cytoplasm",
  "term_id": "GO:0005737",
  "gene_symbol": "POTEI"
}